{
  "term_label": "urea transmembrane transporter activity",
  "gene": "UniProtKB:Q96PS8",
  "gene_name": "Aquaporin-10",
  "gene_symbol": "AQP10",
  "term_id": "GO:0015204"
}